{
  "gene": "UniProtKB:Q9UBD3",
  "term_label": "chemokine-mediated signaling pathway",
  "term_id": "GO:0070098",
  "gene_name": "Cytokine SCM-1 beta",
  "gene_symbol": "XCL2"
}